molecular transducer activity [GO:0060089] (molecular function) Sources: GOC:dos, GOC:pdt Relationships: is a type of molecular_function [GO:0003674] Subtypes: phosphorelay response regulator activity [GO:0000156], GO:0009927, energy transducer activity [GO:0031992], signaling receptor activity [GO:0038023] Definition: A compound molecular function in which an effector function is controlled by one or more regulatory components.